{
  "gene": "UniProtKB:Q9UKA4",
  "term_label": "intracellular protein localization",
  "term_id": "GO:0008104",
  "gene_symbol": "AKAP11",
  "gene_name": "A-kinase anchor protein 11"
}